funalenone catabolic process [GO:1901365] (biological process) Also known as: funalenone breakdown, funalenone catabolism, funalenone degradation Definition: The chemical reactions and pathways resulting in the breakdown of funalenone. Relationships: is a type of phenol-containing compound catabolic process [GO:0019336]; is a type of GO:0042182; is a type of olefinic compound catabolic process [GO:0120256] Sources: GOC:TermGenie, GOC:di